positive regulation of Schwann cell proliferation [GO:0010625] (biological process) Sources: GOC:dph, GOC:sl, GOC:tb Definition: Any process that increases the frequency or rate of the multiplication or reproduction of Schwann cells, resulting in the expansion of their population. Schwann cells are a type of glial cell in the peripheral nervous system. Relationships: is a type of regulation of Schwann cell proliferation [GO:0010624]; is a type of GO:0060252; positively regulates Schwann cell proliferation [GO:0014010] Subtypes: GO:1905046